{
  "gene": "UniProtKB:Q96JQ0",
  "gene_symbol": "DCHS1",
  "term_id": "GO:0016342",
  "term_label": "catenin complex",
  "gene_name": "Protocadherin-16"
}